{
  "gene_symbol": "SEMA3A",
  "term_id": "GO:0005886",
  "gene": "UniProtKB:Q14563",
  "term_label": "plasma membrane",
  "gene_name": "Semaphorin-3A"
}